{
  "gene_symbol": "PHYHIP",
  "term_label": "cytoplasm",
  "gene_name": "Phytanoyl-CoA hydroxylase-interacting protein",
  "term_id": "GO:0005737",
  "gene": "UniProtKB:Q92561"
}